lys-arg specific dibasic protein processing [GO:0090473] (biological process) Sources: GOC:al Relationships: is_a GO:0090472 Definition: Any protein processing achieved by the cleavage of a peptide bond after a lysine-arginine amino acid residue combination within a protein.